{
  "gene_name": "NKG2-A_NKG2-B type II integral membrane protein",
  "gene": "UniProtKB:P26715",
  "term_id": "GO:0009986",
  "term_label": "cell surface",
  "gene_symbol": "KLRC1"
}